arabinan catabolic process [GO:0031222] (biological process) Also known as: arabinan breakdown, arabinan catabolism, arabinan degradation Relationships: is a type of GO:0000272; is a type of arabinan metabolic process [GO:0031221] Sources: GOC:mlg, ISBN:0198506732 Definition: The chemical reactions and pathways resulting in the breakdown of arabinan, a polysaccharide composed of arabinose residues.